{
  "term_id": "GO:0030488",
  "term_label": "tRNA methylation",
  "gene": "UniProtKB:Q53H54",
  "gene_name": "tRNA wybutosine-synthesizing protein 2 homolog",
  "gene_symbol": "TRMT12"
}